{
  "term_label": "actin filament organization",
  "term_id": "GO:0007015",
  "gene_name": "Adenylyl cyclase-associated protein 2",
  "gene": "UniProtKB:P40123",
  "gene_symbol": "CAP2"
}